poly(ribitol phosphate) teichoic acid biosynthetic process [GO:1902012] (biological process) Definition: The chemical reactions and pathways resulting in the formation of poly(ribitol phosphate) teichoic acid. References: PMID:11882717 Sources: GOC:TermGenie, UniPathway:UPA00790 Also known as: poly(ribitol phosphate) teichoic acid anabolism, poly(ribitol phosphate) teichoic acid biosynthesis, poly(ribitol phosphate) teichoic acid formation, poly(ribitol phosphate) teichoic acid synthesis Relationships: is a type of GO:0019350